Hda-beta clamp complex [GO:1990085] (cellular component) Relationships: is a type of replication inhibiting complex [GO:1990078] Also known as: Hda-DnaN complex, Hda-dpo3b complex References: PMID:15150238 Sources: GOC:bhm Definition: A protein complex involved in inactivating the function of DnaA and thereby preventing multiple events of replication initiation. In E. coli, this complex is composed of the beta clamp (DnaN) and Hda.